{
  "gene_name": "Spermatid maturation protein 1",
  "gene_symbol": "SPEM1",
  "term_id": "GO:0007291",
  "gene": "UniProtKB:Q8N4L4",
  "term_label": "sperm individualization"
}